TFIIIB-class transcription factor complex binding [GO:0001154] (molecular function) References: PMID:12381659 Sources: GOC:txnOH Also known as: TFIIIB-class transcription factor binding Relationships: is a type of GO:0001025 Definition: Binding to a general RNA polymerase III transcription factor belonging to the TFIIB complex, one of the factors involved in formation of the preinitiation complex (PIC) by RNA polymerase III.